hemolymph coagulation [GO:0042381] (biological process) Also known as: hemolymph clotting Definition: Any process in which factors in the hemolymph (the invertebrate equivalent of vertebrate blood and lymph) precipitate into insoluble clots in order to prevent loss of body fluid, and at the same time prevent the movement of microbes. Hemolymph coagulation is also part of the invertebrate humoral immune response. References: PMID:10561606, PMID:11915949 Sources: GOC:jl, ISBN:0198506732 Relationships: is a type of humoral immune response [GO:0006959]; is a type of hemostasis [GO:0007599]; is_a GO:0045087; is a type of coagulation [GO:0050817]; is part of GO:0042060